{
  "gene_name": "Ankyrin repeat domain-containing protein 13A",
  "gene_symbol": "ANKRD13A",
  "term_id": "GO:0048259",
  "term_label": "regulation of receptor-mediated endocytosis",
  "gene": "UniProtKB:Q8IZ07"
}